{
  "gene_name": "Methylsterol monooxygenase 1",
  "gene_symbol": "MSMO1",
  "term_id": "GO:0005789",
  "term_label": "endoplasmic reticulum membrane",
  "gene": "UniProtKB:Q15800"
}